{
  "gene_name": "U4_U6.U5 tri-snRNP-associated protein 2",
  "term_id": "UNKNOWN:0003",
  "gene_symbol": "USP39",
  "term_label": "Unknown cellular component",
  "gene": "UniProtKB:Q53GS9"
}